{
  "gene": "UniProtKB:Q8NEV4",
  "term_id": "GO:0032433",
  "gene_symbol": "MYO3A",
  "gene_name": "Myosin-IIIa",
  "term_label": "filopodium tip"
}